cerebral cortex development [GO:0021987] (biological process) Relationships: is a type of anatomical structure development [GO:0048856]; is part of pallium development [GO:0021543] Definition: The progression of the cerebral cortex over time from its initial formation until its mature state. The cerebral cortex is the outer layered region of the telencephalon. Also known as: corticogenesis, neocortex development Sources: GOC:cls, GOC:dgh, GOC:dph, GOC:jid, GO_REF:0000021